{
  "term_id": "GO:0005615",
  "gene_name": "Natriuretic peptides A",
  "gene_symbol": "NPPA",
  "term_label": "extracellular space",
  "gene": "UniProtKB:P01160"
}